{
  "term_id": "GO:0003779",
  "gene_symbol": "MLPH",
  "gene": "UniProtKB:Q9BV36",
  "gene_name": "Melanophilin",
  "term_label": "actin binding"
}